sulfonate dioxygenase activity [GO:0000907] (molecular function) References: PMID:10482536 Sources: GOC:clt Definition: Catalysis of the reaction: sulfonate + 2-oxoglutarate + O2 = sulfite + aminoacetaldehyde + succinate + CO2. Relationships: is a type of 2-oxoglutarate-dependent dioxygenase activity [GO:0016706] Also known as: sulfonate/alpha-ketoglutarate dioxygenase activity, sulphonate dioxygenase activity